{
  "gene_symbol": "ANKRD6",
  "term_id": "UNKNOWN:0003",
  "term_label": "Unknown cellular component",
  "gene_name": "Ankyrin repeat domain-containing protein 6",
  "gene": "UniProtKB:Q9Y2G4"
}